pons morphogenesis [GO:0021583] (BP) Definition: The process in which the anatomical structure of the pons is generated and organized. The pons lies above the medulla and next to the cerebellum. The pons conveys information about movement from the cerebral hemisphere to the cerebellum. Sources: GOC:cls, GOC:dgh, GOC:dph, GOC:jid, GO_REF:0000021 Relationships: is a type of anatomical structure morphogenesis [GO:0009653]; BFO_0000050 pons development [GO:0021548]; is part of hindbrain morphogenesis [GO:0021575]